{
  "term_id": "UNKNOWN:0001",
  "gene_symbol": "COPS4",
  "term_label": "Unknown molecular function",
  "gene": "UniProtKB:Q9BT78",
  "gene_name": "COP9 signalosome complex subunit 4"
}